{
  "term_id": "GO:0030148",
  "gene_symbol": "ELOVL7",
  "gene_name": "Elongation of very long chain fatty acids protein 7",
  "term_label": "sphingolipid biosynthetic process",
  "gene": "UniProtKB:A1L3X0"
}